{
  "term_id": "UNKNOWN:0002",
  "gene_symbol": "GDPD4",
  "gene": "UniProtKB:Q6W3E5",
  "term_label": "Unknown biological process",
  "gene_name": "Glycerophosphodiester phosphodiesterase domain-containing protein 4"
}